{
  "gene_name": "Putative glycine N-acyltransferase-like protein 1B",
  "term_label": "Unknown cellular component",
  "term_id": "UNKNOWN:0003",
  "gene": "UniProtKB:A0A0U1RQE8",
  "gene_symbol": "GLYATL1B"
}